{
  "term_id": "GO:0001822",
  "gene_name": "Cytochrome P450 4A22",
  "gene_symbol": "CYP4A22",
  "gene": "UniProtKB:Q5TCH4",
  "term_label": "kidney development"
}